{
  "term_label": "nucleus",
  "gene": "UniProtKB:O95905",
  "gene_symbol": "ECD",
  "gene_name": "Protein ecdysoneless homolog",
  "term_id": "GO:0005634"
}